{
  "gene_name": "Hydroxyacylglutathione hydrolase-like protein",
  "gene": "UniProtKB:Q6PII5",
  "term_id": "GO:0004416",
  "gene_symbol": "HAGHL",
  "term_label": "hydroxyacylglutathione hydrolase activity"
}